{
  "term_label": "ribonucleoside triphosphate phosphatase activity",
  "term_id": "GO:0017111",
  "gene_symbol": "ENTPD3",
  "gene": "UniProtKB:O75355",
  "gene_name": "Ectonucleoside triphosphate diphosphohydrolase 3"
}